embryonic skeletal joint development [GO:0072498] (BP) Relationships: is a type of GO:0048706 Regulation: regulated by regulation of embryonic skeletal joint development [GO:1902762]; negatively regulated by negative regulation of embryonic skeletal joint development [GO:1902763]; positively regulated by GO:1902764 Definition: The process, occurring during the embryonic phase, whose specific outcome is the progression of the skeletal joints over time, from formation to mature structure. Sources: GOC:BHF, GOC:vk